{
  "gene_symbol": "SLC35A4",
  "term_label": "transmembrane transport",
  "gene": "UniProtKB:Q96G79",
  "gene_name": "Probable UDP-sugar transporter protein SLC35A4",
  "term_id": "GO:0055085"
}